single adenine insertion binding [GO:0032140] (molecular function) Definition: Binding to a double-stranded DNA region containing a single adenine insertion or a deletion that results in an unpaired adenine. Sources: GOC:mah, GOC:vk Relationships: is a type of single base insertion or deletion binding [GO:0032138]